{
  "term_id": "GO:0005634",
  "term_label": "nucleus",
  "gene_symbol": "PROX2",
  "gene": "UniProtKB:Q3B8N5",
  "gene_name": "Prospero homeobox protein 2"
}